{
  "term_label": "Unknown cellular component",
  "term_id": "UNKNOWN:0003",
  "gene_symbol": "PNLIPRP1",
  "gene_name": "Inactive pancreatic lipase-related protein 1",
  "gene": "UniProtKB:P54315"
}